{
  "gene": "UniProtKB:A6H8M9",
  "term_label": "plasma membrane",
  "gene_symbol": "CDHR4",
  "term_id": "GO:0005886",
  "gene_name": "Cadherin-related family member 4"
}